{
  "gene_symbol": "DNAH6",
  "term_id": "GO:0097729",
  "term_label": "9+2 motile cilium",
  "gene": "UniProtKB:Q9C0G6",
  "gene_name": "Dynein axonemal heavy chain 6"
}